{
  "gene_symbol": "TRAV3",
  "gene_name": "T cell receptor alpha variable 3",
  "gene": "UniProtKB:A0A0B4J244",
  "term_label": "immunoglobulin complex",
  "term_id": "GO:0019814"
}